pericentric heterochromatin [GO:0005721] (cellular component) Subtypes: beta-heterochromatin [GO:0005722], alpha-heterochromatin [GO:0005723] Definition: Heterochromatin that is located adjacent to the CENP-A rich centromere 'central core' and characterized by methylated H3 histone at lysine 9 (H3K9me2/H3K9me3). References: PMID:12019236, PMID:20206496, PMID:21437270, PMID:22729156, PMID:9413993 Also known as: centric heterochromatin, centromeric heterochromatin, nuclear centric heterochromatin, nuclear cluster, nuclear pericentric heterochromatin, chromosome, centric outer repeat region, chromosome, centromeric inner repeat region, chromosome, centromeric outer repeat region Relationships: is a type of GO:0000792; is part of chromosome, centromeric region [GO:0000775]